{
  "gene_name": "Inosine-5'-monophosphate dehydrogenase 1",
  "term_label": "IMP dehydrogenase activity",
  "term_id": "GO:0003938",
  "gene": "UniProtKB:P20839",
  "gene_symbol": "IMPDH1"
}